{
  "term_id": "UNKNOWN:0002",
  "gene": "UniProtKB:Q9GZK7",
  "term_label": "Unknown biological process",
  "gene_name": "Olfactory receptor 11A1",
  "gene_symbol": "OR11A1"
}